HUSH2 complex [GO:0140286] (cellular component) Definition: A protein complex that mediates transcriptional silencing of interferon-stimulated genes. In human, it is composed of TASOR2, PPHLN1 and MPHOSPH8. References: PMID:26022416, PMID:39013473, PMID:39489739 Relationships: is a type of GO:0005677